{
  "gene_symbol": "ADCY10",
  "term_id": "GO:0005737",
  "gene_name": "Adenylate cyclase type 10",
  "term_label": "cytoplasm",
  "gene": "UniProtKB:Q96PN6"
}